{
  "gene_symbol": "NAGK",
  "gene_name": "N-acetyl-D-glucosamine kinase",
  "term_label": "Unknown cellular component",
  "gene": "UniProtKB:Q9UJ70",
  "term_id": "UNKNOWN:0003"
}